{
  "gene_symbol": "HMOX1",
  "term_label": "heme catabolic process",
  "gene": "UniProtKB:P09601",
  "gene_name": "Heme oxygenase 1",
  "term_id": "GO:0042167"
}